{
  "gene": "UniProtKB:Q8WWU5",
  "term_label": "acrosomal vesicle",
  "term_id": "GO:0001669",
  "gene_symbol": "TCP11",
  "gene_name": "T-complex protein 11 homolog"
}